regulation of branching involved in lung morphogenesis [GO:0061046] (biological process) Relationships: is a type of regulation of morphogenesis of a branching structure [GO:0060688]; is_a GO:1905330; regulates GO:0060441 Sources: GOC:dph, GOC:yaf Subtypes: lung induction [GO:0060492], positive regulation of branching involved in lung morphogenesis [GO:0061047], GO:0061048 Definition: Any process that modulates the rate, frequency, or extent of the process in which a highly ordered sequence of patterning events generates the branched structures of the lung, consisting of reiterated combinations of bud outgrowth, elongation, and dichotomous subdivision of terminal units.